post-anaphase array microtubule [GO:1905759] (cellular component) Relationships: is a type of GO:0005874; is part of GO:1990295 Also known as: microtubule of PAA, microtubule of post-anaphase array, microtubule of post-anaphase microtubule array, microtubuli of PAA, microtubuli of post-anaphase array, microtubuli of post-anaphase microtubule array, microtubulus of PAA, microtubulus of post-anaphase array, microtubulus of post-anaphase microtubule array, neurotubule of PAA, neurotubule of post-anaphase array, neurotubule of post-anaphase microtubule array Definition: Any microtubule that is part of a post-anaphase microtubule array. References: PMID:11007487 Sources: GOC:TermGenie, GO_REF:0000064